{
  "gene": "UniProtKB:A6NJ08",
  "gene_name": "Putative methyl-CpG-binding domain protein 3-like 5",
  "gene_symbol": "MBD3L5",
  "term_label": "negative regulation of transcription by RNA polymerase II",
  "term_id": "GO:0000122"
}